vesicle organization [GO:0016050] (biological process) Also known as: vesicle organisation, vesicle organization and biogenesis Sources: GOC:mah Subtypes: phagolysosome assembly [GO:0001845], vesicle budding from membrane [GO:0006900], vesicle coating [GO:0006901], vesicle fusion [GO:0006906], GO:0007032, synaptic vesicle maturation [GO:0016188], contractile vacuole organization [GO:0033298], GO:0033363, pigment granule organization [GO:0048753], GO:0071255, extracellular exosome assembly [GO:0071971], GO:1902900, GO:1905556 Relationships: is a type of organelle organization [GO:0006996] Definition: A process that is carried out at the cellular level which results in the assembly, arrangement of constituent parts, or disassembly of a vesicle.